vinorine hydroxylase activity [GO:0050596] (molecular function) Sources: EC:1.14.14.104, RHEA:17257 Relationships: is a type of GO:0016709 Definition: Catalysis of the reaction: H+ + NADPH + O2 + vinorine = H2O + NADP+ + vomilenine. Also known as: vinorine,NADPH:oxygen oxidoreductase (21alpha-hydroxylating)